{
  "gene_symbol": "HGS",
  "gene_name": "Hepatocyte growth factor-regulated tyrosine kinase substrate",
  "term_label": "receptor internalization",
  "term_id": "GO:0031623",
  "gene": "UniProtKB:O14964"
}